phenylacetyl-CoA dehydrogenase activity [GO:0033789] (molecular function) Relationships: is a type of oxidoreductase activity, acting on CH or CH2 groups, quinone or similar compound as acceptor [GO:0033695] Sources: RHEA:15705 Definition: Catalysis of the reaction: 2 1,4-benzoquinone + H2O + phenylacetyl-CoA = 2 hydroquinone + phenylglyoxylyl-CoA. Also known as: phenylacetyl-CoA:acceptor oxidoreductase activity, phenylacetyl-CoA:quinone oxidoreductase activity